regulation of interleukin-13 production [GO:0032656] (biological process) Also known as: regulation of IL-13 production, regulation of interleukin-13 biosynthetic process, regulation of interleukin-13 secretion Relationships: is_a GO:0001817; regulates interleukin-13 production [GO:0032616] Sources: GOC:mah Definition: Any process that modulates the frequency, rate, or extent of interleukin-13 production. Subtypes: negative regulation of interleukin-13 production [GO:0032696], positive regulation of interleukin-13 production [GO:0032736]